{
  "gene": "UniProtKB:Q8NI77",
  "term_label": "ATP hydrolysis activity",
  "gene_symbol": "KIF18A",
  "gene_name": "Kinesin-like protein KIF18A",
  "term_id": "GO:0016887"
}